{
  "term_id": "GO:0032982",
  "term_label": "myosin filament",
  "gene_symbol": "MYH3",
  "gene": "UniProtKB:P11055",
  "gene_name": "Myosin-3"
}